{
  "term_label": "axon",
  "gene_symbol": "COMT",
  "gene": "UniProtKB:P21964",
  "term_id": "GO:0030424",
  "gene_name": "Catechol O-methyltransferase"
}